{
  "term_label": "protein tyrosine phosphatase activity",
  "term_id": "GO:0004725",
  "gene_name": "Dual specificity protein phosphatase 22",
  "gene_symbol": "DUSP22",
  "gene": "UniProtKB:Q9NRW4"
}